pigment granule organization [GO:0048753] (biological process) Sources: GOC:rc Also known as: pigment granule organisation, pigment granule organization and biogenesis Relationships: is a type of GO:0016050; BFO_0000050 cellular pigmentation [GO:0033059] Subtypes: eye pigment granule organization [GO:0008057], ocellus pigment granule organization [GO:0008058], melanosome organization [GO:0032438] Definition: A process that is carried out at the cellular level which results in the assembly, arrangement of constituent parts, or disassembly of a pigment granule.